{
  "term_label": "netrin receptor activity",
  "gene": "UniProtKB:Q6UXZ4",
  "gene_name": "Netrin receptor UNC5D",
  "term_id": "GO:0005042",
  "gene_symbol": "UNC5D"
}